{
  "term_id": "GO:0033617",
  "term_label": "mitochondrial respiratory chain complex IV assembly",
  "gene": "UniProtKB:Q8N8Q8",
  "gene_symbol": "COX18",
  "gene_name": "Cytochrome c oxidase assembly protein COX18, mitochondrial"
}